neuron apoptotic process [GO:0051402] (biological process) Definition: Any apoptotic process in a neuron, the basic cellular unit of nervous tissue. Each neuron consists of a body, an axon, and dendrites. Their purpose is to receive, conduct, and transmit impulses in the nervous system. Relationships: is_a apoptotic process [GO:0006915] Regulation: regulated by regulation of neuron apoptotic process [GO:0043523]; negatively regulated by negative regulation of neuron apoptotic process [GO:0043524]; positively regulated by positive regulation of neuron apoptotic process [GO:0043525] Also known as: apoptosis of neuronal cells, apoptosis of neurons, neuron programmed cell death by apoptosis, neuronal cell apoptosis, neuronal cell programmed cell death by apoptosis, programmed cell death of neuronal cells by apoptosis, programmed cell death of neurons by apoptosis, programmed cell death, neuronal cells, programmed cell death, neurons, neuron apoptosis Sources: CL:0000540, GOC:mtg_apoptosis Subtypes: motor neuron apoptotic process [GO:0097049], retinal rod cell apoptotic process [GO:0097473], retinal cone cell apoptotic process [GO:0097474], GO:0110088, outer hair cell apoptotic process [GO:1905584]